{
  "gene_symbol": "SLC11A2",
  "term_id": "GO:0015094",
  "gene_name": "Natural resistance-associated macrophage protein 2",
  "term_label": "lead ion transmembrane transporter activity",
  "gene": "UniProtKB:P49281"
}